{
  "term_label": "nucleoplasm",
  "term_id": "GO:0005654",
  "gene_name": "Homeobox protein Hox-C4",
  "gene": "UniProtKB:P09017",
  "gene_symbol": "HOXC4"
}